laminin-5 complex [GO:0005610] (cellular component) Relationships: is a type of laminin complex [GO:0043256] References: PMID:10842354 Sources: GOC:jl Also known as: laminin-3A32 complex, laminin-5A complex, laminin-332 complex Definition: A laminin complex composed of alpha3, beta3 and gamma2 polypeptide chains.